{
  "gene_name": "Coronin-1C",
  "term_label": "actin filament",
  "gene_symbol": "CORO1C",
  "gene": "UniProtKB:Q9ULV4",
  "term_id": "GO:0005884"
}